 [go#goslim:euk:cellular:processes:ribbon] Note: GO ribbon for eukaroytic cellular processes